{
  "term_label": "innate immune response",
  "term_id": "GO:0045087",
  "gene_symbol": "TRIM51G",
  "gene": "UniProtKB:A0A3B3IT33",
  "gene_name": "Putative tripartite motif-containing protein 51G"
}